{
  "gene_symbol": "CNOT3",
  "term_id": "UNKNOWN:0001",
  "gene_name": "CCR4-NOT transcription complex subunit 3",
  "gene": "UniProtKB:O75175",
  "term_label": "Unknown molecular function"
}